{
  "term_id": "GO:0006974",
  "term_label": "DNA damage response",
  "gene_name": "Serine_threonine-protein kinase VRK2",
  "gene_symbol": "VRK2",
  "gene": "UniProtKB:Q86Y07"
}